{
  "gene": "UniProtKB:Q8N9V7",
  "term_id": "UNKNOWN:0001",
  "term_label": "Unknown molecular function",
  "gene_name": "Protein TOPAZ1",
  "gene_symbol": "TOPAZ1"
}